{
  "term_label": "nucleus",
  "gene_symbol": "ZFP82",
  "term_id": "GO:0005634",
  "gene_name": "Zinc finger protein 82 homolog",
  "gene": "UniProtKB:Q8N141"
}